regulation of post-transcriptional gene silencing by regulatory ncRNA [GO:1900368] (biological process) Relationships: is a type of regulation of post-transcriptional gene silencing [GO:0060147]; is a type of regulation of gene silencing by regulatory ncRNA [GO:0060966]; RO_0002211 regulatory ncRNA-mediated post-transcriptional gene silencing [GO:0035194] Subtypes: GO:0060964, negative regulation of post-transcriptional gene silencing by regulatory ncRNA [GO:1900369], positive regulation of post-transcriptional gene silencing by RNA [GO:1900370] Also known as: regulation of PTGS, regulation of RNA interference, regulation of RNAi, regulation of post-transcriptional gene silencing by RNA, regulation of post-transcriptional gene silencing by ncRNA Definition: Any process that modulates the frequency, rate or extent of post-transcriptional gene silencing by a non-coding RNA. References: PMID:22412382 Sources: GOC:TermGenie, GOC:kmv